{
  "term_label": "dehydroascorbic acid transport",
  "term_id": "GO:0070837",
  "gene": "UniProtKB:P11166",
  "gene_name": "Solute carrier family 2, facilitated glucose transporter member 1",
  "gene_symbol": "SLC2A1"
}